{
  "gene": "UniProtKB:P13164",
  "gene_symbol": "IFITM1",
  "gene_name": "Interferon-induced transmembrane protein 1",
  "term_id": "GO:0060337",
  "term_label": "type I interferon-mediated signaling pathway"
}